{
  "term_label": "protein secretion",
  "term_id": "GO:0009306",
  "gene_symbol": "TVP23C",
  "gene": "UniProtKB:Q96ET8",
  "gene_name": "Golgi apparatus membrane protein TVP23 homolog C"
}